{
  "gene_name": "Kinesin-like protein KIF26A",
  "term_label": "regulation of neuron migration",
  "term_id": "GO:2001222",
  "gene_symbol": "KIF26A",
  "gene": "UniProtKB:Q9ULI4"
}